{
  "term_label": "extracellular region",
  "gene_symbol": "FSTL5",
  "term_id": "GO:0005576",
  "gene_name": "Follistatin-related protein 5",
  "gene": "UniProtKB:Q8N475"
}